nucleobase catabolic process [GO:0046113] (biological process) Subtypes: purine nucleobase catabolic process [GO:0006145], GO:0006208 Definition: The chemical reactions and pathways resulting in the breakdown of a nucleobase, a nitrogenous base that is a constituent of a nucleic acid. Sources: GOC:ai Also known as: nucleobase breakdown, nucleobase catabolism, nucleobase degradation Relationships: is a type of GO:0009056; is a type of nucleobase metabolic process [GO:0009112]